{
  "term_label": "regulation of mRNA splicing, via spliceosome",
  "term_id": "GO:0048024",
  "gene_symbol": "SON",
  "gene_name": "Protein SON",
  "gene": "UniProtKB:P18583"
}